L-cysteine catabolic process [GO:0019448] (biological process) Definition: The chemical reactions and pathways resulting in the breakdown of L-cysteine, the L-enantiomer of 2-amino-3-mercaptopropanoic acid, i.e. (2R)-2-amino-3-mercaptopropanoic acid. Subtypes: GO:0019449, L-cysteine catabolic process to pyruvate [GO:0019450], L-cysteine catabolic process to taurine [GO:0019452], GO:0019453 Also known as: L-cysteine breakdown, L-cysteine catabolism, L-cysteine degradation Sources: GOC:jsg, GOC:mah Relationships: is_a cysteine catabolic process [GO:0009093]; is a type of L-cysteine metabolic process [GO:0046439]; is a type of L-amino acid catabolic process [GO:0170035]; is a type of proteinogenic amino acid catabolic process [GO:0170040]